{
  "gene_name": "Bifunctional heparan sulfate N-deacetylase_N-sulfotransferase 4",
  "term_label": "Golgi apparatus",
  "term_id": "GO:0005794",
  "gene": "UniProtKB:Q9H3R1",
  "gene_symbol": "NDST4"
}